poly-ADP-D-ribose binding [GO:0072572] (molecular function) Relationships: is a type of carbohydrate derivative binding [GO:0097367] References: PMID:20088964 Sources: GOC:mah, GOC:sart Also known as: poly-ADP-ribose binding, pADPr binding Definition: Binding to polymeric ADP-D-ribose, a polymer that is composed of poly-ADP-D-ribose units linked through 1,2-glycosidic bonds at the ribose ring.